positive regulation of pericentric heterochromatin formation [GO:0090053] (biological process) Sources: GOC:dph, GOC:tb Relationships: is a type of positive regulation of heterochromatin formation [GO:0031453]; is a type of GO:0090052; positively regulates pericentric heterochromatin formation [GO:0031508] Definition: Any process that increases the frequency, rate or extent of pericentric heterochromatin formation. Also known as: positive regulation of chromatin silencing at centromere, positive regulation of pericentric heterochromatin assembly